{
  "gene_symbol": "CHRNA2",
  "term_id": "GO:0099171",
  "gene_name": "Neuronal acetylcholine receptor subunit alpha-2",
  "gene": "UniProtKB:Q15822",
  "term_label": "presynaptic modulation of chemical synaptic transmission"
}